{
  "term_label": "mitochondrion",
  "gene_name": "Large ribosomal subunit protein mL45",
  "term_id": "GO:0005739",
  "gene_symbol": "MRPL45",
  "gene": "UniProtKB:Q9BRJ2"
}